{
  "gene_symbol": "TRAJ43",
  "term_label": "Unknown cellular component",
  "gene_name": "T cell receptor alpha joining 43 (Fragment)",
  "gene": "UniProtKB:A0A075B6V1",
  "term_id": "UNKNOWN:0003"
}